{
  "term_id": "UNKNOWN:0002",
  "gene_symbol": "NWD2",
  "term_label": "Unknown biological process",
  "gene": "UniProtKB:Q9ULI1",
  "gene_name": "NACHT and WD repeat domain-containing protein 2"
}